{
  "gene_name": "Novel acetylcholine receptor chaperone",
  "term_id": "GO:0005783",
  "gene": "UniProtKB:Q53FP2",
  "term_label": "endoplasmic reticulum",
  "gene_symbol": "TMEM35A"
}